{
  "gene_symbol": "INF2",
  "gene": "UniProtKB:Q27J81",
  "term_label": "actin filament",
  "gene_name": "Inverted formin-2",
  "term_id": "GO:0005884"
}